{
  "gene_name": "Ly6_PLAUR domain-containing protein 6B",
  "term_id": "GO:0030548",
  "gene": "UniProtKB:Q8NI32",
  "term_label": "acetylcholine receptor regulator activity",
  "gene_symbol": "LYPD6B"
}